{
  "gene_symbol": "IGHV4-59",
  "term_id": "GO:0016064",
  "term_label": "immunoglobulin mediated immune response",
  "gene": "UniProtKB:P01825",
  "gene_name": "Immunoglobulin heavy variable 4-59"
}